{
  "gene_name": "Protein FEV",
  "term_label": "cell differentiation",
  "gene": "UniProtKB:Q99581",
  "term_id": "GO:0030154",
  "gene_symbol": "FEV"
}